endoplasmic reticulum tubular network membrane organization [GO:1990809] (biological process) Definition: A process that is carried out at the cellular level which results in the assembly, arrangement of constituent parts, or disassembly of the endoplasmic reticulum (ER) tubular network membrane. References: PMID:20434336 Relationships: is a type of endoplasmic reticulum tubular network organization [GO:0071786]; is a type of endoplasmic reticulum membrane organization [GO:0090158]